{
  "gene_symbol": "PNMA3",
  "gene_name": "Paraneoplastic antigen Ma3",
  "term_label": "Unknown cellular component",
  "term_id": "UNKNOWN:0003",
  "gene": "UniProtKB:Q9UL41"
}